{
  "gene_name": "Mitotic checkpoint protein BUB3",
  "term_id": "GO:0033597",
  "gene": "UniProtKB:O43684",
  "term_label": "mitotic checkpoint complex",
  "gene_symbol": "BUB3"
}